{
  "term_label": "nucleus",
  "gene": "UniProtKB:P27361",
  "gene_symbol": "MAPK3",
  "gene_name": "Mitogen-activated protein kinase 3",
  "term_id": "GO:0005634"
}